{
  "gene": "UniProtKB:P33981",
  "term_id": "GO:0005634",
  "gene_name": "Dual specificity protein kinase TTK",
  "gene_symbol": "TTK",
  "term_label": "nucleus"
}